{
  "gene_symbol": "MUC1",
  "term_label": "apical plasma membrane",
  "term_id": "GO:0016324",
  "gene_name": "Mucin-1",
  "gene": "UniProtKB:P15941"
}